negative regulation of glucocorticoid catabolic process [GO:0031950] (biological process) Definition: Any process that stops, prevents, or reduces the frequency, rate or extent of the chemical reactions and pathways resulting in the breakdown of glucocorticoids. Relationships: is a type of regulation of glucocorticoid catabolic process [GO:0031949]; is a type of negative regulation of steroid metabolic process [GO:0045939]; is a type of negative regulation of lipid catabolic process [GO:0050995]; negatively regulates glucocorticoid catabolic process [GO:0006713] Also known as: down regulation of glucocorticoid catabolic process, down-regulation of glucocorticoid catabolic process, downregulation of glucocorticoid catabolic process, inhibition of glucocorticoid catabolic process Sources: GOC:mah